{
  "term_id": "GO:0140410",
  "gene": "UniProtKB:Q9ULF5",
  "term_label": "monoatomic cation:bicarbonate symporter activity",
  "gene_name": "Zinc transporter ZIP10",
  "gene_symbol": "SLC39A10"
}